{
  "term_id": "GO:0007608",
  "gene_symbol": "OMP",
  "gene": "UniProtKB:P47874",
  "term_label": "sensory perception of smell",
  "gene_name": "Olfactory marker protein"
}